DNA insertion or deletion binding [GO:0032135] (molecular function) Subtypes: heteroduplex DNA loop binding [GO:0000404], single base insertion or deletion binding [GO:0032138], dinucleotide insertion or deletion binding [GO:0032139] Relationships: is a type of mismatched DNA binding [GO:0030983] Definition: Binding to a double-stranded DNA region containing an insertion or a deletion. Also known as: insertion binding, DNA insertion binding Sources: GOC:vk